{
  "gene": "UniProtKB:Q9NVM4",
  "term_label": "histone methyltransferase activity",
  "gene_symbol": "PRMT7",
  "gene_name": "Protein arginine N-methyltransferase 7",
  "term_id": "GO:0042054"
}